{
  "term_id": "GO:0005783",
  "gene": "UniProtKB:O76096",
  "gene_name": "Cystatin-F",
  "gene_symbol": "CST7",
  "term_label": "endoplasmic reticulum"
}